positive regulation of lipid kinase activity [GO:0090218] (biological process) Sources: GOC:dph, GOC:tb Definition: Any process that increases the frequency, rate or extent of lipid kinase activity, the catalysis of the transfer of a phosphate group, usually from ATP, to a simple or complex lipid. Relationships: is a type of positive regulation of kinase activity [GO:0033674]; is a type of regulation of lipid kinase activity [GO:0043550]; is a type of positive regulation of lipid metabolic process [GO:0045834]; positively regulates GO:0001727